{
  "gene_name": "V-set and transmembrane domain-containing protein 5",
  "term_label": "filopodium assembly",
  "gene": "UniProtKB:A8MXK1",
  "term_id": "GO:0046847",
  "gene_symbol": "VSTM5"
}